{
  "gene": "UniProtKB:Q09472",
  "gene_name": "Histone acetyltransferase p300",
  "gene_symbol": "EP300",
  "term_id": "GO:0003713",
  "term_label": "transcription coactivator activity"
}